retinal bipolar neuron differentiation [GO:0060040] (biological process) Definition: The process in which a relatively unspecialized cell acquires specialized features of a bipolar cell, the last neuron to be generated in the retina. Sources: GOC:ascb_2009, GOC:bf, GOC:dph, GOC:tb Relationships: is_a glutamatergic neuron differentiation [GO:1905962]; BFO_0000050 neural retina development [GO:0003407]; is part of retina morphogenesis in camera-type eye [GO:0060042] Subtypes: rod bipolar cell differentiation [GO:1904389], cone retinal bipolar cell differentiation [GO:1904390]